{
  "gene": "UniProtKB:P42658",
  "term_label": "plasma membrane",
  "gene_symbol": "DPP6",
  "term_id": "GO:0005886",
  "gene_name": "Dipeptidyl aminopeptidase-like protein 6"
}